chemokine (C-X-C motif) ligand 2 production [GO:0072567] (biological process) Definition: The appearance of chemokine (C-X-C motif) ligand 2 due to biosynthesis or secretion following a cellular stimulus, resulting in an increase in its intracellular or extracellular levels. Regulation: regulated by regulation of chemokine (C-X-C motif) ligand 2 production [GO:2000341]; negatively regulated by GO:2000342; positively regulated by GO:2000343 Also known as: CXCL2 production, MIP-2 production, MIP2 production, SCYB2 production Sources: GOC:BHF, GOC:mah Relationships: is_a chemokine production [GO:0032602]